{
  "gene_name": "C-type lectin domain family 1 member A",
  "term_label": "transmembrane signaling receptor activity",
  "gene_symbol": "CLEC1A",
  "term_id": "GO:0004888",
  "gene": "UniProtKB:Q8NC01"
}